vitamin-K-epoxide reductase (warfarin-sensitive) activity [GO:0047057] (molecular function) Relationships: is a type of oxidoreductase activity, acting on CH or CH2 groups, disulfide as acceptor [GO:0016728] Also known as: vitamin K1 epoxide reductase activity, phylloquinone epoxide reductase activity Definition: Catalysis of the reaction: phylloquinol + a protein with a disulfide bond = phylloquinone + a protein with reduced L-cysteine residues. Sources: RHEA:57744